{
  "term_id": "GO:0003730",
  "gene_name": "RNA-binding motif, single-stranded-interacting protein 3",
  "term_label": "mRNA 3'-UTR binding",
  "gene_symbol": "RBMS3",
  "gene": "UniProtKB:Q6XE24"
}